{
  "gene": "UniProtKB:Q6UXF1",
  "term_label": "retrograde axonal transport",
  "term_id": "GO:0008090",
  "gene_symbol": "TMEM108",
  "gene_name": "Transmembrane protein 108"
}